{
  "gene_symbol": "SLC22A13",
  "term_label": "Unknown biological process",
  "term_id": "UNKNOWN:0002",
  "gene": "UniProtKB:Q9Y226",
  "gene_name": "Solute carrier family 22 member 13"
}